{
  "term_id": "GO:0051864",
  "gene_name": "Bifunctional peptidase and arginyl-hydroxylase JMJD5",
  "term_label": "histone H3K36 demethylase activity",
  "gene_symbol": "KDM8",
  "gene": "UniProtKB:Q8N371"
}